{
  "term_label": "calmodulin binding",
  "gene_name": "GTP-binding protein Rit1",
  "gene_symbol": "RIT1",
  "term_id": "GO:0005516",
  "gene": "UniProtKB:Q92963"
}